{
  "term_id": "GO:0008198",
  "gene_symbol": "ACP5",
  "gene_name": "Tartrate-resistant acid phosphatase type 5",
  "term_label": "ferrous iron binding",
  "gene": "UniProtKB:P13686"
}